toxin activity [GO:0090729] (molecular function) Definition: Interacting selectively with one or more biological molecules in another (target) organism, initiating pathogenesis (leading to an abnormal, generally detrimental state) in the target organism. The activity should refer to an evolved function of the active gene product, i.e. one that was selected for. Examples include the activity of botulinum toxin, and snake venom. Sources: GOC:pt Relationships: is a type of molecular_function [GO:0003674]; is part of modulation of process of another organism [GO:0035821] Also known as: toxin receptor binding